{
  "term_label": "cortical cytoskeleton",
  "gene": "UniProtKB:O15511",
  "gene_symbol": "ARPC5",
  "gene_name": "Actin-related protein 2_3 complex subunit 5",
  "term_id": "GO:0030863"
}